protein-arginine omega-N asymmetric methyltransferase activity [GO:0035242] (molecular function) Note: Note that type I protein arginine N-methyltransferase enzymes possess 'protein-arginine omega-N monomethyltransferase activity ; GO:0035241' and 'protein-arginine omega-N asymmetric methyltransferase activity ; GO:0035242'. Also known as: protein arginine omega-N asymmetric methylase activity, protein arginine omega-N asymmetric methyltransferase activity, S-adenosyl-L-methionine:[protein]-L-arginine N-methyltransferase ([protein]-Nomega,Nomega-dimethyl-L-arginine-forming), type I PRMT activity, type I protein arginine methyltransferase activity References: PMID:14705965 Definition: Catalysis of the addition of a second methyl group to methylated peptidyl-arginine. Methylation is on the same terminal nitrogen (omega nitrogen) residue that was previously methylated, resulting in asymmetrical peptidyl-N(omega),N(omega)-dimethylated arginine residues. Relationships: is a type of GO:0016274